{
  "term_label": "calcium ion binding",
  "gene_symbol": "CIB4",
  "term_id": "GO:0005509",
  "gene_name": "Calcium and integrin-binding family member 4",
  "gene": "UniProtKB:A0PJX0"
}